{
  "gene_symbol": "CLDN11",
  "term_label": "bicellular tight junction",
  "gene_name": "Claudin-11",
  "term_id": "GO:0005923",
  "gene": "UniProtKB:O75508"
}